folic acid binding [GO:0005542] (molecular function) Relationships: is a type of vitamin binding [GO:0019842]; is a type of carboxylic acid binding [GO:0031406]; is a type of amide binding [GO:0033218]; is a type of modified amino acid binding [GO:0072341]; is a type of GO:1901363 Sources: GOC:jl, ISBN:0198506732 Definition: Binding to folic acid, pteroylglutamic acid. Folic acid is widely distributed as a member of the vitamin B complex and is essential for the synthesis of purine and pyrimidines. Also known as: folate binding, vitamin B9 binding, vitamin M binding